{
  "term_id": "UNKNOWN:0003",
  "term_label": "Unknown cellular component",
  "gene_symbol": "UPB1",
  "gene": "UniProtKB:Q9UBR1",
  "gene_name": "Beta-ureidopropionase"
}